{
  "gene_symbol": "PPP1R14B",
  "term_id": "GO:0045087",
  "term_label": "innate immune response",
  "gene_name": "Protein phosphatase 1 regulatory subunit 14B",
  "gene": "UniProtKB:Q96C90"
}